{
  "gene_symbol": "RAN",
  "gene": "UniProtKB:P62826",
  "gene_name": "GTP-binding nuclear protein Ran",
  "term_id": "GO:0005737",
  "term_label": "cytoplasm"
}